{
  "gene_symbol": "STEAP1B",
  "gene": "UniProtKB:Q6NZ63",
  "gene_name": "STEAP family member 1B",
  "term_id": "GO:0005768",
  "term_label": "endosome"
}